{
  "gene_name": "Dual specificity protein phosphatase CDC14C",
  "gene_symbol": "CDC14C",
  "term_label": "cytoplasm",
  "term_id": "GO:0005737",
  "gene": "UniProtKB:A4D256"
}